oxidoreductase activity, acting on the CH-CH group of donors, cytochrome as acceptor [GO:0016632] (molecular function) Subtypes: galactonolactone dehydrogenase activity [GO:0016633], GO:0080049 Relationships: is a type of oxidoreductase activity, acting on the CH-CH group of donors [GO:0016627] Sources: EC:1.3.2.- Definition: Catalysis of an oxidation-reduction (redox) reaction in which a CH-CH group acts as a hydrogen or electron donor and reduces a cytochrome.